{
  "term_id": "GO:0005829",
  "gene_name": "Myeloid cell nuclear differentiation antigen",
  "gene_symbol": "MNDA",
  "term_label": "cytosol",
  "gene": "UniProtKB:P41218"
}